{
  "gene": "UniProtKB:O43633",
  "term_label": "endosome transport via multivesicular body sorting pathway",
  "gene_name": "Charged multivesicular body protein 2a",
  "term_id": "GO:0032509",
  "gene_symbol": "CHMP2A"
}